{
  "term_label": "cellular response to unfolded protein",
  "gene": "UniProtKB:Q9UJY1",
  "gene_symbol": "HSPB8",
  "term_id": "GO:0034620",
  "gene_name": "Heat shock protein beta-8"
}